{
  "gene_symbol": "NCAPD2",
  "term_label": "condensed chromosome, centromeric region",
  "gene": "UniProtKB:Q15021",
  "gene_name": "Condensin complex subunit 1",
  "term_id": "GO:0000779"
}